{
  "gene_symbol": "HAP1",
  "term_id": "GO:0017022",
  "gene_name": "Huntingtin-associated protein 1",
  "gene": "UniProtKB:P54257",
  "term_label": "myosin binding"
}